{
  "term_label": "ciliary basal body",
  "gene_symbol": "TTLL7",
  "gene_name": "Tubulin polyglutamylase TTLL7",
  "gene": "UniProtKB:Q6ZT98",
  "term_id": "GO:0036064"
}